{
  "gene_name": "Serine_threonine-protein kinase Nek7",
  "gene": "UniProtKB:Q8TDX7",
  "term_label": "nucleus",
  "gene_symbol": "NEK7",
  "term_id": "GO:0005634"
}